{
  "gene_name": "Insulin-like growth factor 2 mRNA-binding protein 1",
  "gene_symbol": "IGF2BP1",
  "term_label": "cytoplasm",
  "gene": "UniProtKB:Q9NZI8",
  "term_id": "GO:0005737"
}